{
  "term_id": "GO:0044613",
  "term_label": "nuclear pore central transport channel",
  "gene_symbol": "NUTF2",
  "gene_name": "Nuclear transport factor 2",
  "gene": "UniProtKB:P61970"
}